{
  "gene": "UniProtKB:P69892",
  "gene_symbol": "HBG2",
  "term_id": "GO:0005833",
  "term_label": "hemoglobin complex",
  "gene_name": "Hemoglobin subunit gamma-2"
}